{
  "gene": "UniProtKB:Q96T49",
  "gene_name": "Protein phosphatase 1 regulatory inhibitor subunit 16B",
  "term_label": "cytoplasm",
  "gene_symbol": "PPP1R16B",
  "term_id": "GO:0005737"
}